{
  "gene_name": "Protein unc-80 homolog",
  "term_label": "cation channel complex",
  "gene": "UniProtKB:Q8N2C7",
  "term_id": "GO:0034703",
  "gene_symbol": "UNC80"
}